inositol tetrakisphosphate phosphatase activity [GO:0052743] (MF) Definition: Catalysis of the reaction: myo-inositol tetrakisphosphate + H2O = myo-inositol trisphosphate + phosphate. Sources: GOC:ai Relationships: is a type of GO:0052745 Subtypes: inositol-1,4,5,6-tetrakisphosphate 6-phosphatase activity [GO:0030352], GO:0051717, inositol-1,3,4,5-tetrakisphosphate 5-phosphatase activity [GO:0052659], inositol-1,3,4,6-tetrakisphosphate 6-phosphatase activity [GO:0052830], inositol-1,3,4,6-tetrakisphosphate 1-phosphatase activity [GO:0052831], inositol-1,2,4,5-tetrakisphosphate 5-phosphatase activity [GO:1990649], inositol-2,4,5,6-tetrakisphosphate 5-phosphatase activity [GO:1990650]